{
  "term_label": "BMP signaling pathway",
  "gene": "UniProtKB:Q9NR23",
  "gene_name": "Growth_differentiation factor 3",
  "gene_symbol": "GDF3",
  "term_id": "GO:0030509"
}